small nucleolar ribonucleoprotein complex assembly [GO:0000491] (biological process) Also known as: snoRNP assembly Relationships: is a type of protein-RNA complex assembly [GO:0022618] Subtypes: box C/D snoRNP assembly [GO:0000492], box H/ACA snoRNP assembly [GO:0000493] Sources: GOC:krc Definition: The aggregation, arrangement and bonding together of proteins and a snoRNA to form a small nucleolar ribonucleoprotein (snoRNP) complex.